sperm karyosome formation [GO:0061989] (biological process) Definition: The chromosome organization process in which meiotic chromosomes in the spem nucleus cluster together to form a compact spherical structure called the karyosome. Relationships: is a type of karyosome formation [GO:0061988]; is part of GO:0007283 References: PMID:19696886